{
  "gene_name": "Putative sodium-coupled neutral amino acid transporter 10",
  "term_id": "GO:0016020",
  "gene_symbol": "SLC38A10",
  "gene": "UniProtKB:Q9HBR0",
  "term_label": "membrane"
}